{
  "gene": "UniProtKB:Q9P2D7",
  "term_id": "GO:0051959",
  "gene_name": "Dynein axonemal heavy chain 1",
  "gene_symbol": "DNAH1",
  "term_label": "dynein light intermediate chain binding"
}